DnaB-DnaC-Rep-PriC complex [GO:1990160] (cellular component) Relationships: is a type of pre-primosome complex [GO:1990099]; has part GO:1990100 References: PMID:19941825, PMID:8663105 Sources: GOC:bhm Also known as: DnaB-DnaC-Rep-PriC preprimosome, phi-X174-type preprimosome Definition: A protein-DNA complex consisting of the helicase loading complex DnaB-DnaC, replication restart proteins Rep and PriC, and associated DNA. Involved in the restart of DNA replication after a stalled replication fork has been repaired.